{
  "gene_symbol": "NELFB",
  "gene": "UniProtKB:Q8WX92",
  "term_label": "NELF complex",
  "gene_name": "Negative elongation factor B",
  "term_id": "GO:0032021"
}